{
  "term_id": "GO:0004888",
  "term_label": "transmembrane signaling receptor activity",
  "gene_symbol": "TREM1",
  "gene": "UniProtKB:Q9NP99",
  "gene_name": "Triggering receptor expressed on myeloid cells 1"
}